{
  "gene_symbol": "SASS6",
  "gene_name": "Spindle assembly abnormal protein 6 homolog",
  "term_label": "centrosome",
  "gene": "UniProtKB:Q6UVJ0",
  "term_id": "GO:0005813"
}